{
  "gene": "UniProtKB:Q9BZJ0",
  "gene_name": "Crooked neck-like protein 1",
  "gene_symbol": "CRNKL1",
  "term_id": "GO:0000245",
  "term_label": "spliceosomal complex assembly"
}